{
  "gene_name": "Abasic site processing protein HMCES",
  "gene_symbol": "HMCES",
  "term_label": "single-stranded DNA binding",
  "gene": "UniProtKB:Q96FZ2",
  "term_id": "GO:0003697"
}